bulk synaptic vesicle endocytosis [GO:0150008] (BP) Definition: Endocytosis of large regions of presynaptic membrane after intense stimulation-mediated fusion of multiple synaptic vesicles. Bulk endocytosis is triggered by high loads of membrane addition through exocytosis of synaptic vesicles and elevated concentration of calcium in the presynapse. References: PMID:18250322, PMID:18579735, PMID:19266323, PMID:26430111, PMID:28391090 Sources: GOC:aruk, GOC:bc, GOC:ha Relationships: is a type of synaptic vesicle endocytosis [GO:0048488] Also known as: ADBE, activity-dependent bulk endocytosis, activity-dependent bulk synaptic vesicle endocytosis, bulk endocytosis